{
  "gene_name": "TM2 domain-containing protein 3",
  "gene_symbol": "TM2D3",
  "term_id": "UNKNOWN:0002",
  "gene": "UniProtKB:Q9BRN9",
  "term_label": "Unknown biological process"
}